{
  "term_id": "GO:0015203",
  "gene_name": "Polyamine-transporting ATPase 13A3",
  "gene_symbol": "ATP13A3",
  "term_label": "polyamine transmembrane transporter activity",
  "gene": "UniProtKB:Q9H7F0"
}